{
  "gene_name": "Nuclear pore complex-interacting protein family member B7",
  "gene_symbol": "NPIPB7",
  "term_label": "Unknown cellular component",
  "gene": "UniProtKB:O75200",
  "term_id": "UNKNOWN:0003"
}